{
  "gene": "UniProtKB:Q15223",
  "term_label": "plasma membrane",
  "term_id": "GO:0005886",
  "gene_name": "Nectin-1",
  "gene_symbol": "NECTIN1"
}